limb development [GO:0060173] (biological process) Relationships: is a type of appendage development [GO:0048736] Definition: The process whose specific outcome is the progression of a limb over time, from its formation to the mature structure. A limb is an appendage of an animal used for locomotion or grasping. Examples include legs, arms or some types of fin. Also known as: paired limb/fin development, limb bud development References: PMID:11487378 Sources: GOC:dgh, GOC:dph Subtypes: pectoral fin development [GO:0033339], pelvic fin development [GO:0033340]